MHC protein complex assembly [GO:0002396] (BP) References: PMID:15771591, PMID:15928678 Sources: GOC:add, ISBN:0781735149 Subtypes: MHC class I protein complex assembly [GO:0002397], MHC class Ib protein complex assembly [GO:0002398], GO:0002399 Relationships: is a type of protein-containing complex assembly [GO:0065003] Definition: The aggregation, arrangement and bonding together of a set of components to form an MHC protein complex.